pronephros structural organization [GO:0072118] (biological process) Relationships: is a type of anatomical structure arrangement [GO:0048532]; is part of pronephros morphogenesis [GO:0072114] Sources: GOC:mtg_kidney_jan10 Subtypes: head kidney structural organization [GO:0072119] Also known as: pronephric kidney structural organization, pronephros structural organisation Definition: The process that contributes to the act of creating the structural organization of the pronephros. This process pertains to the physical shaping of a rudimentary structure. In mammals, the pronephros is the first of the three embryonic kidneys to be established and exists only transiently. In lower vertebrates such as fish and amphibia, the pronephros is the fully functional embryonic kidney and is indispensable for larval life.